{
  "term_label": "ubiquitin-dependent protein catabolic process",
  "term_id": "GO:0006511",
  "gene": "UniProtKB:Q7Z419",
  "gene_symbol": "RNF144B",
  "gene_name": "E3 ubiquitin-protein ligase RNF144B"
}